pentose catabolic process [GO:0019323] (biological process) Relationships: is a type of GO:0019321; is a type of monosaccharide catabolic process [GO:0046365] Definition: The chemical reactions and pathways resulting in the breakdown of a pentose, any monosaccharide with a chain of five carbon atoms in the molecule. Subtypes: xylulose catabolic process [GO:0005998], D-ribose catabolic process [GO:0019303], arabinose catabolic process [GO:0019568], D-xylose catabolic process [GO:0042843] Also known as: pentose breakdown, pentose catabolism, pentose degradation Sources: ISBN:0198506732